{
  "gene_name": "Protocadherin gamma-B2",
  "gene": "UniProtKB:Q9Y5G2",
  "term_id": "GO:0005886",
  "gene_symbol": "PCDHGB2",
  "term_label": "plasma membrane"
}